{
  "term_label": "U12-type spliceosomal complex",
  "gene_symbol": "SNRPG",
  "term_id": "GO:0005689",
  "gene": "UniProtKB:P62308",
  "gene_name": "Small nuclear ribonucleoprotein G"
}